{
  "term_id": "UNKNOWN:0003",
  "term_label": "Unknown cellular component",
  "gene_name": "Immunoglobulin heavy variable 1-45",
  "gene_symbol": "IGHV1-45",
  "gene": "UniProtKB:A0A0A0MS14"
}